{
  "gene": "UniProtKB:Q9P206",
  "gene_symbol": "NHSL3",
  "term_label": "cell differentiation",
  "gene_name": "Uncharacterized protein KIAA1522",
  "term_id": "GO:0030154"
}